{
  "gene_name": "Leukemia inhibitory factor",
  "gene_symbol": "LIF",
  "term_id": "GO:0005615",
  "term_label": "extracellular space",
  "gene": "UniProtKB:P15018"
}